4-amino-4-deoxychorismate lyase activity [GO:0008696] (molecular function) Also known as: aminodeoxychorismate lyase activity, 4-amino-4-deoxychorismate pyruvate-lyase (4-aminobenzoate-forming), 4-amino-4-deoxychorismate pyruvate-lyase activity, ADC lyase activity, enzyme X activity, p-aminobenzoate synthetase, para-aminobenzoic acid (PABA) synthase, para-aminobenzoic acid synthase Definition: Catalysis of the reaction: 4-amino-4-deoxychorismate = 4-aminobenzoate + H+ + pyruvate. Relationships: is a type of oxo-acid-lyase activity [GO:0016833] Note: Note that the name 'para-amino benzoic acid synthase' was initially given to the 'aminodeoxychorismate synthase' activity before the additional 4-amino-4-deoxychorismate lyase activity was discovered. It is the lyase activity that actually produces para-aminobenzoic acid from 4-amino-4-deoxychorismate. Sources: EC:4.1.3.38, RHEA:16201